{
  "term_id": "UNKNOWN:0003",
  "gene_symbol": "ASMT",
  "gene_name": "Acetylserotonin O-methyltransferase",
  "gene": "UniProtKB:P46597",
  "term_label": "Unknown cellular component"
}